{
  "gene_symbol": "ZSCAN32",
  "gene": "UniProtKB:Q9NX65",
  "term_id": "UNKNOWN:0003",
  "term_label": "Unknown cellular component",
  "gene_name": "Zinc finger and SCAN domain-containing protein 32"
}